{
  "gene_symbol": "TRBV7-6",
  "gene": "UniProtKB:A0A1B0GX31",
  "term_id": "UNKNOWN:0001",
  "term_label": "Unknown molecular function",
  "gene_name": "T cell receptor beta variable 7-6"
}